polythionate oxidation [GO:0019416] (biological process) Sources: MetaCyc:THIOSULFOX-PWY Relationships: is a type of GO:0006790 Definition: The chemical reactions and pathways resulting in the conversion of thiosulfate to tetrathionate, using cytochrome c as an electron acceptor.